3-hydroxyindolin-2-one monooxygenase activity [GO:0036192] (molecular function) Relationships: is a type of oxidoreductase activity, acting on paired donors, with incorporation or reduction of molecular oxygen, reduced flavin or flavoprotein as one donor, and incorporation of one atom of oxygen [GO:0016712] Sources: RHEA:31927 Definition: Catalysis of the reaction: 3-hydroxyindolin-2-one + O2 + reduced [NADPH--hemoprotein reductase] = 2-hydroxy-2H-1,4-benzoxazin-3(4H)-one + H+ + H2O + oxidized [NADPH--hemoprotein reductase]. Also known as: 3-hydroxyindolin-2-one,NAD(P)H:oxygen oxidoreductase (2-hydroxy-2H-1,4-benzoxazin-3(4H)-one-forming)